{
  "gene_symbol": "ELP6",
  "term_label": "elongator holoenzyme complex",
  "gene": "UniProtKB:Q0PNE2",
  "gene_name": "Elongator complex protein 6",
  "term_id": "GO:0033588"
}